{
  "gene": "UniProtKB:P55899",
  "term_label": "external side of plasma membrane",
  "gene_name": "IgG receptor FcRn large subunit p51",
  "term_id": "GO:0009897",
  "gene_symbol": "FCGRT"
}